positive regulation of amino acid metabolic process [GO:0045764] (biological process) Also known as: positive regulation of amino acid metabolism, positive regulation of cellular amino acid metabolic process, up regulation of amino acid metabolic process, up-regulation of amino acid metabolic process, upregulation of amino acid metabolic process, activation of amino acid metabolic process, stimulation of amino acid metabolic process Sources: GOC:go_curators Subtypes: positive regulation of L-tryptophan metabolic process [GO:0090358], positive regulation of tetrapyrrole biosynthetic process from glutamate [GO:1901412], positive regulation of tetrapyrrole biosynthetic process from glycine and succinyl-CoA [GO:1901415], GO:1901717, positive regulation of ornithine catabolic process [GO:1903268], GO:2000284, positive regulation of L-proline catabolic process to L-glutamate [GO:2001158], positive regulation of ammonia assimilation cycle [GO:2001250] Definition: Any process that activates or increases the frequency, rate or extent of the chemical reactions and pathways involving amino acid. Relationships: is a type of GO:0006521; is a type of positive regulation of metabolic process [GO:0009893]; positively regulates amino acid metabolic process [GO:0006520]